carbon catabolite repression of transcription by glucose [GO:0045014] (biological process) Definition: A transcription regulation process in which the presence of glucose leads to a decrease in the frequency, rate, or extent of transcription of specific genes involved in the metabolism of other carbon sources. Carbon catabolite repression is a mechanism of genetic regulation which the accumulation of catabolites of one substance in the cell represses the formation of enzymes that contribute to the catabolism of other substances. References: PMID:11018147 Sources: ISBN:0198506732 Also known as: down regulation of transcription by glucose, down-regulation of transcription by glucose, downregulation of transcription by glucose, glucose effect, glucose repression, inhibition of transcription by glucose Relationships: is a type of carbon catabolite repression of transcription [GO:0045013]; is a type of negative regulation of transcription by glucose [GO:0061986] Subtypes: carbon catabolite repression of transcription from RNA polymerase II promoter by glucose [GO:0000433]